{
  "gene_symbol": "SETMAR",
  "gene_name": "Histone-lysine N-methyltransferase SETMAR",
  "term_label": "nucleus",
  "gene": "UniProtKB:Q53H47",
  "term_id": "GO:0005634"
}